tripeptide import across plasma membrane [GO:0140207] (biological process) References: PMID:22226946 Relationships: is_a tripeptide transmembrane transport [GO:0035443]; is a type of oligopeptide import across plasma membrane [GO:0140205] Subtypes: glutathione import across plasma membrane [GO:0098709] Definition: The directed movement of a tripeptide from outside of a cell, across the plasma membrane and into the cytosol.